{
  "gene": "UniProtKB:P35813",
  "gene_symbol": "PPM1A",
  "gene_name": "Protein phosphatase 1A",
  "term_label": "nucleus",
  "term_id": "GO:0005634"
}